{
  "gene_symbol": "TUBA3E",
  "term_label": "GTP binding",
  "gene_name": "Tubulin alpha-3E chain",
  "gene": "UniProtKB:Q6PEY2",
  "term_id": "GO:0005525"
}